{
  "term_id": "UNKNOWN:0001",
  "gene_symbol": "SLITRK5",
  "gene": "UniProtKB:O94991",
  "gene_name": "SLIT and NTRK-like protein 5",
  "term_label": "Unknown molecular function"
}